positive regulation of fibroblast growth factor receptor signaling pathway [GO:0045743] (biological process) Also known as: positive regulation of FGF receptor signaling pathway, positive regulation of FGF receptor signalling pathway, positive regulation of FGFR signaling pathway, up regulation of fibroblast growth factor receptor signaling pathway, up-regulation of fibroblast growth factor receptor signaling pathway, upregulation of fibroblast growth factor receptor signaling pathway, activation of fibroblast growth factor receptor signaling pathway, stimulation of fibroblast growth factor receptor signaling pathway Relationships: is a type of GO:0009967; is a type of regulation of fibroblast growth factor receptor signaling pathway [GO:0040036]; positively regulates GO:0008543 Subtypes: positive regulation of fibroblast growth factor receptor signaling pathway involved in neural plate anterior/posterior pattern formation [GO:2000315], positive regulation of fibroblast growth factor receptor signaling pathway involved in ureteric bud formation [GO:2000704] Sources: GOC:go_curators Definition: Any process that activates or increases the frequency, rate or extent of fibroblast growth factor receptor signaling pathway activity.